{
  "gene_name": "Guanine nucleotide-binding protein G(t) subunit alpha-2",
  "gene_symbol": "GNAT2",
  "term_label": "adenylate cyclase-modulating G protein-coupled receptor signaling pathway",
  "term_id": "GO:0007188",
  "gene": "UniProtKB:P19087"
}